{
  "term_id": "UNKNOWN:0001",
  "gene": "UniProtKB:A0A0A6YYD4",
  "gene_symbol": "TRBV13",
  "gene_name": "T cell receptor beta variable 13",
  "term_label": "Unknown molecular function"
}